{
  "gene_name": "Coiled-coil domain-containing protein 91",
  "term_id": "UNKNOWN:0001",
  "gene": "UniProtKB:Q7Z6B0",
  "term_label": "Unknown molecular function",
  "gene_symbol": "CCDC91"
}